{
  "gene": "UniProtKB:P02775",
  "term_label": "chemokine activity",
  "term_id": "GO:0008009",
  "gene_name": "Platelet basic protein",
  "gene_symbol": "PPBP"
}